{
  "gene_name": "Nuclear pore complex protein Nup133",
  "gene_symbol": "NUP133",
  "term_id": "GO:0016973",
  "term_label": "poly(A)+ mRNA export from nucleus",
  "gene": "UniProtKB:Q8WUM0"
}